rRNA (guanine-N1-)-methyltransferase activity [GO:0008989] (molecular function) Also known as: S-adenosyl-L-methionine:rRNA (guanine-1-N-)-methyltransferase activity, ribosomal ribonucleate guanine 1-methyltransferase activity, S-adenosyl-L-methionine:rRNA (guanine-N1-)-methyltransferase activity Subtypes: GO:0052911, 23S rRNA (guanine(748)-N(1))-methyltransferase activity [GO:0052912] Definition: Catalysis of the reaction: S-adenosyl-L-methionine + rRNA = S-adenosyl-L-homocysteine + rRNA containing N1-methylguanine. Relationships: is a type of N-methyltransferase activity [GO:0008170]; is a type of rRNA (guanine) methyltransferase activity [GO:0016435] Sources: GOC:curators